{
  "gene_name": "C-C chemokine receptor type 5",
  "gene_symbol": "CCR5",
  "term_id": "GO:0006954",
  "gene": "UniProtKB:P51681",
  "term_label": "inflammatory response"
}